{
  "gene": "UniProtKB:Q9HCT0",
  "gene_name": "Fibroblast growth factor 22",
  "term_label": "positive regulation of cell population proliferation",
  "gene_symbol": "FGF22",
  "term_id": "GO:0008284"
}